{
  "term_id": "GO:0045892",
  "term_label": "negative regulation of DNA-templated transcription",
  "gene_name": "BTB_POZ domain-containing protein KCTD15",
  "gene_symbol": "KCTD15",
  "gene": "UniProtKB:Q96SI1"
}